positive regulation of positive thymic T cell selection [GO:1902234] (biological process) Also known as: positive regulation of positive thymic T lymphocyte selection, positive regulation of positive thymic T-cell selection, positive regulation of positive thymic T-lymphocyte selection, up regulation of positive thymic T cell selection, up regulation of positive thymic T lymphocyte selection, up regulation of positive thymic T-cell selection, up regulation of positive thymic T-lymphocyte selection, up-regulation of positive thymic T cell selection, up-regulation of positive thymic T lymphocyte selection, up-regulation of positive thymic T-cell selection, up-regulation of positive thymic T-lymphocyte selection, upregulation of positive thymic T cell selection, upregulation of positive thymic T lymphocyte selection, upregulation of positive thymic T-cell selection, upregulation of positive thymic T-lymphocyte selection, activation of positive thymic T cell selection, activation of positive thymic T lymphocyte selection, activation of positive thymic T-cell selection, activation of positive thymic T-lymphocyte selection Relationships: is a type of positive regulation of T cell differentiation in thymus [GO:0033089]; is a type of GO:1902232; positively regulates positive thymic T cell selection [GO:0045059] References: PMID:22080863 Sources: GOC:TermGenie Definition: Any process that activates or increases the frequency, rate or extent of positive thymic T cell selection.